positive regulation of establishment of protein-containing complex localization to telomere [GO:1904915] (biological process) Also known as: positive regulation of establishment of macromolecular complex localisation to telomere, up regulation of establishment of macromolecular complex localisation to telomere, up regulation of establishment of macromolecular complex localization to telomere, up-regulation of establishment of macromolecular complex localisation to telomere, up-regulation of establishment of macromolecular complex localization to telomere, upregulation of establishment of macromolecular complex localisation to telomere, upregulation of establishment of macromolecular complex localization to telomere, activation of establishment of macromolecular complex localisation to telomere, activation of establishment of macromolecular complex localization to telomere, positive regulation of establishment of macromolecular complex localization to telomere Definition: Any process that activates or increases the frequency, rate or extent of establishment of the localization of a protein-containing macromolecular complex to a telomere. Relationships: is_a GO:0048518; is a type of regulation of establishment of protein-containing complex localization to telomere [GO:1904913]; positively regulates establishment of protein-containing complex localization to telomere [GO:0097695] References: PMID:26586433 Sources: GOC:BHF, GOC:BHF_telomere, GOC:TermGenie, GOC:rph, GO_REF:0000058